{
  "term_label": "all-trans retinal 3,4-desaturase activity",
  "gene": "UniProtKB:Q4G0S4",
  "gene_symbol": "CYP27C1",
  "gene_name": "Cytochrome P450 27C1",
  "term_id": "GO:0061897"
}